{
  "gene_name": "Zinc finger protein 660",
  "gene": "UniProtKB:Q6AZW8",
  "gene_symbol": "ZNF660",
  "term_id": "GO:0000978",
  "term_label": "RNA polymerase II cis-regulatory region sequence-specific DNA binding"
}